{
  "gene_symbol": "ZNF598",
  "term_label": "Unknown cellular component",
  "gene_name": "E3 ubiquitin-protein ligase ZNF598",
  "term_id": "UNKNOWN:0003",
  "gene": "UniProtKB:Q86UK7"
}